{
  "gene": "UniProtKB:Q8IWT1",
  "term_label": "cardiac conduction",
  "gene_symbol": "SCN4B",
  "gene_name": "Sodium channel subunit beta-4",
  "term_id": "GO:0061337"
}